{
  "gene_symbol": "FCHO2",
  "term_id": "UNKNOWN:0001",
  "gene": "UniProtKB:Q0JRZ9",
  "term_label": "Unknown molecular function",
  "gene_name": "F-BAR domain only protein 2"
}